{
  "term_id": "UNKNOWN:0001",
  "term_label": "Unknown molecular function",
  "gene_symbol": "CAVIN4",
  "gene_name": "Caveolae-associated protein 4",
  "gene": "UniProtKB:Q5BKX8"
}